regulation of microvillus assembly [GO:0032534] (biological process) Subtypes: negative regulation of microvillus assembly [GO:1903697], positive regulation of microvillus assembly [GO:1903698] Also known as: regulation of microvillus biogenesis Definition: A process that modulates the formation of a microvillus. Relationships: is a type of regulation of microvillus organization [GO:0032530]; is a type of regulation of plasma membrane bounded cell projection assembly [GO:0120032]; regulates microvillus assembly [GO:0030033] Sources: GOC:mah